{
  "term_label": "transmembrane receptor protein tyrosine kinase activity",
  "gene": "UniProtKB:Q04912",
  "gene_symbol": "MST1R",
  "gene_name": "Macrophage-stimulating protein receptor",
  "term_id": "GO:0004714"
}